{
  "term_id": "GO:0140693",
  "gene": "UniProtKB:Q6ZQX7",
  "gene_name": "Protein LIAT1",
  "gene_symbol": "LIAT1",
  "term_label": "molecular condensate scaffold activity"
}